{
  "gene_name": "CREB-regulated transcription coactivator 2",
  "gene_symbol": "CRTC2",
  "gene": "UniProtKB:Q53ET0",
  "term_id": "GO:0045944",
  "term_label": "positive regulation of transcription by RNA polymerase II"
}